{
  "term_id": "GO:0009755",
  "term_label": "hormone-mediated signaling pathway",
  "gene_name": "Thyrotropin receptor",
  "gene": "UniProtKB:P16473",
  "gene_symbol": "TSHR"
}